{
  "term_id": "GO:1903981",
  "gene": "UniProtKB:P02768",
  "term_label": "enterobactin binding",
  "gene_symbol": "ALB",
  "gene_name": "Albumin"
}